optic nerve formation [GO:0021634] (BP) Sources: GOC:cls, GOC:dgh, GOC:dph, GOC:jid, GO_REF:0000021 Definition: The process that gives rise to the optic nerve. This process pertains to the initial formation of a structure from unspecified parts. The sensory optic nerve originates from the bipolar cells of the retina and conducts visual information to the brainstem. The optic nerve exits the back of the eye in the orbit, enters the optic canal, and enters the central nervous system at the optic chiasm (crossing) where the nerve fibers become the optic tract just prior to entering the hindbrain. Also known as: CN II biosynthesis, CN II formation Relationships: is a type of GO:0021603; is part of optic nerve morphogenesis [GO:0021631] Regulation: regulated by regulation of optic nerve formation [GO:2000595]; RO_0002212 by GO:2000596; positively regulated by positive regulation of optic nerve formation [GO:2000597]